{
  "gene_symbol": "C11orf40",
  "gene_name": "Putative uncharacterized protein C11orf40",
  "term_id": "UNKNOWN:0002",
  "term_label": "Unknown biological process",
  "gene": "UniProtKB:Q8WZ69"
}